{
  "gene_name": "Hemicentin-1",
  "term_id": "GO:0005886",
  "term_label": "plasma membrane",
  "gene_symbol": "HMCN1",
  "gene": "UniProtKB:Q96RW7"
}